{
  "gene_name": "Homeobox protein CDX-1",
  "term_label": "RNA polymerase II transcription regulatory region sequence-specific DNA binding",
  "gene_symbol": "CDX1",
  "term_id": "GO:0000977",
  "gene": "UniProtKB:P47902"
}